response to pheromone regulating pheromone-induced unidirectional conjugation [GO:0000765] (biological process) Definition: Any process that results in a change in state or activity of a cell or an organism (in terms of movement, secretion, enzyme production, gene expression, etc.) as a result of a pheromone stimulus that regulates the process of pheromone-induced unidirectional conjugation. Sources: GOC:clt Also known as: response to pheromone during pheromone-induced unidirectional Relationships: is a type of GO:0019236; regulates pheromone-induced unidirectional conjugation [GO:0000762]